{
  "gene_symbol": "ZNF501",
  "gene_name": "Zinc finger protein 501",
  "term_label": "regulation of transcription by RNA polymerase II",
  "gene": "UniProtKB:Q96CX3",
  "term_id": "GO:0006357"
}